neurotransmitter receptor internalization [GO:0099590] (biological process) Relationships: is a type of receptor internalization [GO:0031623] Definition: A receptor-mediated endocytosis process that results in the internalization of a neurotransmitter receptor. Subtypes: postsynaptic neurotransmitter receptor internalization [GO:0098884] Sources: GOC:dos